{
  "term_label": "steroid catabolic process",
  "gene_name": "Cytochrome P450 1B1",
  "gene": "UniProtKB:Q16678",
  "gene_symbol": "CYP1B1",
  "term_id": "GO:0006706"
}